{
  "gene_name": "Inositol-3-phosphate synthase 1",
  "gene_symbol": "ISYNA1",
  "term_id": "GO:0005737",
  "gene": "UniProtKB:Q9NPH2",
  "term_label": "cytoplasm"
}